{
  "term_label": "Unknown molecular function",
  "term_id": "UNKNOWN:0001",
  "gene": "UniProtKB:P0DMU7",
  "gene_name": "Cancer_testis antigen family 45 member A6",
  "gene_symbol": "CT45A6"
}